{
  "gene_name": "Phospholipid scramblase 3",
  "gene": "UniProtKB:Q9NRY6",
  "term_id": "GO:0090199",
  "gene_symbol": "PLSCR3",
  "term_label": "regulation of release of cytochrome c from mitochondria"
}